quercetin-3-sulfate 3'-sulfotransferase activity [GO:0047365] (molecular function) Relationships: is a type of sulfotransferase activity [GO:0008146] Sources: EC:2.8.2.26, RHEA:22504 Definition: Catalysis of the reaction: 3'-phospho-5'-adenylyl sulfate + quercetin 3-sulfate = adenosine 3',5'-diphosphate + H+ + quercetin 3,3'-disulfate. Also known as: quercetin-3-sulphate 3'-sulphotransferase activity, 3'-phosphoadenylyl-sulfate:quercetin-3-sulfate 3'-sulfotransferase activity, 3'-sulfotransferase activity, PAPS:flavonol 3-sulfate 3'-sulfotransferase activity, flavonol 3'-sulfotransferase activity